{
  "gene_name": "D-aminoacyl-tRNA deacylase 1",
  "gene_symbol": "DTD1",
  "gene": "UniProtKB:Q8TEA8",
  "term_id": "GO:0006399",
  "term_label": "tRNA metabolic process"
}